root system development [GO:0022622] (BP) Definition: The process whose specific outcome is the progression of the root system over time, from its formation to the mature structure. Sources: GOC:isa_complete Relationships: is a type of system development [GO:0048731]